{
  "gene": "UniProtKB:Q8TE49",
  "gene_symbol": "OTUD7A",
  "gene_name": "OTU domain-containing protein 7A",
  "term_label": "nucleus",
  "term_id": "GO:0005634"
}